{
  "gene_symbol": "MYH10",
  "term_label": "actomyosin structure organization",
  "gene": "UniProtKB:P35580",
  "term_id": "GO:0031032",
  "gene_name": "Myosin-10"
}